{
  "gene_symbol": "NOP2",
  "term_id": "GO:0009383",
  "gene": "UniProtKB:P46087",
  "gene_name": "Probable 28S rRNA (cytosine(4447)-C(5))-methyltransferase",
  "term_label": "rRNA (cytosine-C5-)-methyltransferase activity"
}